negative regulation of 18-methylnonadec-1-ene biosynthetic process [GO:1900951] (biological process) Definition: Any process that stops, prevents or reduces the frequency, rate or extent of 18-methylnonadec-1-ene biosynthetic process. Sources: GOC:TermGenie, GOC:mengo_curators Also known as: down regulation of 18-methylnonadec-1-ene anabolism, down regulation of 18-methylnonadec-1-ene biosynthesis, down regulation of 18-methylnonadec-1-ene biosynthetic process, down regulation of 18-methylnonadec-1-ene formation, down regulation of 18-methylnonadec-1-ene synthesis, down-regulation of 18-methylnonadec-1-ene anabolism, down-regulation of 18-methylnonadec-1-ene biosynthesis, down-regulation of 18-methylnonadec-1-ene biosynthetic process, down-regulation of 18-methylnonadec-1-ene formation, down-regulation of 18-methylnonadec-1-ene synthesis, downregulation of 18-methylnonadec-1-ene anabolism, downregulation of 18-methylnonadec-1-ene biosynthesis, downregulation of 18-methylnonadec-1-ene biosynthetic process, downregulation of 18-methylnonadec-1-ene formation, downregulation of 18-methylnonadec-1-ene synthesis, inhibition of 18-methylnonadec-1-ene anabolism, inhibition of 18-methylnonadec-1-ene biosynthesis, inhibition of 18-methylnonadec-1-ene formation, inhibition of 18-methylnonadec-1-ene synthesis, negative regulation of 18-methylnonadec-1-ene anabolism, negative regulation of 18-methylnonadec-1-ene biosynthesis, negative regulation of 18-methylnonadec-1-ene formation, negative regulation of 18-methylnonadec-1-ene synthesis, inhibition of 18-methylnonadec-1-ene biosynthetic process Relationships: is a type of negative regulation of olefin biosynthetic process [GO:1900912]; is a type of GO:1900950; negatively regulates 18-methylnonadec-1-ene biosynthetic process [GO:1900881]